{
  "gene": "UniProtKB:O60636",
  "term_id": "UNKNOWN:0002",
  "term_label": "Unknown biological process",
  "gene_name": "Tetraspanin-2",
  "gene_symbol": "TSPAN2"
}